{
  "gene": "UniProtKB:Q6NZ36",
  "term_label": "K63-linked polyubiquitin modification-dependent protein binding",
  "gene_name": "Fanconi anemia core complex-associated protein 20",
  "term_id": "GO:0070530",
  "gene_symbol": "FAAP20"
}